{
  "gene_name": "Vesicle transport protein SEC20",
  "gene": "UniProtKB:Q12981",
  "term_label": "retrograde vesicle-mediated transport, Golgi to endoplasmic reticulum",
  "gene_symbol": "BNIP1",
  "term_id": "GO:0006890"
}